sodium:ammonium:chloride symporter activity [GO:7770002] (molecular function) Definition: Enables the transfer of a solute or solutes from one side of a membrane to the other according to the reaction: Na+(out) + NH4+(out) + Cl-(out) = Na+(in) + NH4+(in) + Cl-(in). Relationships: is a type of GO:0015378 References: PMID:12657561